embryonic digestive tract development [GO:0048566] (biological process) Relationships: is a type of digestive tract development [GO:0048565]; is a type of embryonic organ development [GO:0048568] Definition: The process whose specific outcome is the progression of the gut over time, from its formation to the mature structure during embryonic development. The gut is the region of the digestive tract extending from the beginning of the intestines to the anus. Subtypes: GO:0048611 Sources: GOC:go_curators